{
  "gene_name": "Inactive L-threonine 3-dehydrogenase, mitochondrial",
  "term_id": "UNKNOWN:0003",
  "term_label": "Unknown cellular component",
  "gene_symbol": "TDH",
  "gene": "UniProtKB:Q8IZJ6"
}